{
  "term_id": "GO:0030594",
  "gene_name": "Histamine H4 receptor",
  "gene_symbol": "HRH4",
  "term_label": "neurotransmitter receptor activity",
  "gene": "UniProtKB:Q9H3N8"
}